{
  "gene_name": "Proteasome subunit beta type-4",
  "gene_symbol": "PSMB4",
  "gene": "UniProtKB:P28070",
  "term_label": "nucleus",
  "term_id": "GO:0005634"
}